{
  "gene_symbol": "TSC22D2",
  "gene": "UniProtKB:O75157",
  "term_label": "Unknown molecular function",
  "term_id": "UNKNOWN:0001",
  "gene_name": "TSC22 domain family protein 2"
}